{
  "gene_name": "NCK-interacting protein with SH3 domain",
  "gene_symbol": "NCKIPSD",
  "term_id": "GO:0071933",
  "gene": "UniProtKB:Q9NZQ3",
  "term_label": "Arp2/3 complex binding"
}